phosphatidylcholine:diacylglycerol cholinephosphotransferase activity [GO:0102249] (molecular function) Relationships: is a type of GO:0016780 Sources: GOC:pz, MetaCyc:RXN-12386 Definition: Catalysis of the reaction: a phosphatidylcholine + a 1,2-diacyl-sn-glycerol = a 1,2-diacyl-sn-glycerol + a phosphatidylcholine.